{
  "gene_symbol": "DNAJC2",
  "gene": "UniProtKB:Q99543",
  "gene_name": "DnaJ homolog subfamily C member 2",
  "term_id": "GO:0043022",
  "term_label": "ribosome binding"
}